COPI coating of Golgi vesicle [GO:0048205] (biological process) Relationships: is a type of Golgi transport vesicle coating [GO:0048200]; is part of COPI-coated vesicle budding [GO:0035964] Definition: The addition of COPI proteins and adaptor proteins to Golgi membranes during the formation of transport vesicles, forming a vesicle coat. References: PMID:10219233 Sources: GOC:jid, GOC:mah, ISBN:0716731363 Subtypes: COPI coating of Golgi vesicle, inter-Golgi cisterna [GO:0010787], COPI coating of Golgi vesicle, cis-Golgi to rough ER [GO:0010788] Also known as: COPI coating of Golgi-derived vesicle, COPI vesicle coating